tRNA N1-guanine methylation [GO:0002939] (biological process) Sources: ISBN:155581073X, ISBN:1555811337 Definition: The process whereby a guanine in tRNA is methylated at position N1 of the guanine. Also known as: tRNA m1-guanine biosynthesis Relationships: is a type of tRNA methylation [GO:0030488]